{
  "term_id": "UNKNOWN:0001",
  "gene_symbol": "A0A087WUM9",
  "gene_name": "Uncharacterized protein",
  "gene": "UniProtKB:A0A087WUM9",
  "term_label": "Unknown molecular function"
}